{
  "term_label": "Unknown biological process",
  "gene": "UniProtKB:O15347",
  "term_id": "UNKNOWN:0002",
  "gene_name": "High mobility group protein B3",
  "gene_symbol": "HMGB3"
}